{
  "gene_name": "Plastin-3",
  "term_id": "GO:0005737",
  "gene_symbol": "PLS3",
  "gene": "UniProtKB:P13797",
  "term_label": "cytoplasm"
}